negative regulation of leukocyte migration [GO:0002686] (biological process) Relationships: is a type of negative regulation of immune system process [GO:0002683]; is a type of GO:0002685; is a type of negative regulation of cell migration [GO:0030336]; negatively regulates GO:0050900 Sources: GOC:add Also known as: down regulation of leukocyte migration, down-regulation of leukocyte migration, downregulation of leukocyte migration, negative regulation of immune cell migration, negative regulation of leucocyte migration, inhibition of leukocyte migration Subtypes: GO:0002689, negative regulation of cellular extravasation [GO:0002692], negative regulation of mononuclear cell migration [GO:0071676], GO:1902623, negative regulation of eosinophil migration [GO:2000417] Definition: Any process that stops, prevents, or reduces the frequency, rate, or extent of leukocyte migration.